{
  "term_id": "GO:0002376",
  "gene": "UniProtKB:Q13568",
  "gene_symbol": "IRF5",
  "term_label": "immune system process",
  "gene_name": "Interferon regulatory factor 5"
}